ERBB3:ERBB2 complex [GO:0038143] (cellular component) Relationships: is a type of plasma membrane signaling receptor complex [GO:0098802] Definition: A heterodimeric complex between the tyrosine kinase receptor ERBB2 and a ligand-activated receptor ERBB3. ERBB2, which does not bind any known ligand, is activated through formation of a heterodimer with another ligand-activated ERBB family member such as ERBB3. Also known as: EGFR:ERBB2 heterodimer, NRG1/2:ERBB3:ERBB2 References: PMID:16460914, PMID:8665853 Sources: GOC:signaling